{
  "gene": "UniProtKB:A0A7I2V4U8",
  "term_id": "UNKNOWN:0002",
  "gene_name": "Uncharacterized protein",
  "term_label": "Unknown biological process",
  "gene_symbol": "A0A7I2V4U8"
}